response to nocodazole [GO:1904402] (biological process) Definition: Any process that results in a change in state or activity of a cell or an organism (in terms of movement, secretion, enzyme production, gene expression, etc.) as a result of a nocodazole stimulus. Subtypes: GO:1904403 References: PMID:17822405 Sources: GOC:TermGenie, GO_REF:0000071 Relationships: is a type of GO:1901654; is_a GO:1901698